coenzyme F420H2:quinone oxidoreductase activity [GO:0052755] (molecular function) Relationships: is a type of oxidoreductase activity, acting on CH-OH group of donors [GO:0016614] References: PMID:10971593, PMID:8055920 Sources: RHEA:39663 Definition: Catalysis of the reaction: oxidized coenzyme F420-(gamma-L-Glu)(n) + a quinol + H+ = reduced coenzyme F420-(gamma-L-Glu)(n) + a quinone. Also known as: F420H2-dependent quinone oxidoreductase activity, F420H2:2,3-dimethyl-1,4-naphthoquinone oxidoreductase activity, F420H2:quinone oxidoreductase activity, reduced coenzyme F420:quinone oxidoreductase activity